regulation of formation of growth cone in injured axon [GO:1905942] (biological process) References: PMID:19737525 Sources: GOC:TermGenie, GO_REF:0000058 Subtypes: negative regulation of formation of growth cone in injured axon [GO:1905943], GO:1905944 Definition: Any process that modulates the frequency, rate or extent of formation of growth cone in injured axon. Relationships: is a type of GO:0048686; regulates formation of growth cone in injured axon [GO:0048689]